{
  "gene": "UniProtKB:Q9Y5S1",
  "gene_symbol": "TRPV2",
  "term_id": "GO:0098703",
  "term_label": "calcium ion import across plasma membrane",
  "gene_name": "Transient receptor potential cation channel subfamily V member 2"
}